epithelial cell proliferation involved in liver morphogenesis [GO:0072575] (biological process) Sources: GOC:BHF, GOC:mah Relationships: is a type of epithelial cell proliferation [GO:0050673]; is part of liver morphogenesis [GO:0072576] Subtypes: hepatocyte proliferation [GO:0072574] Definition: The multiplication or reproduction of epithelial cells, resulting in the expansion of a cell population that contributes to the shaping of the liver.